radial glia guided migration of Purkinje cell [GO:0021942] (biological process) References: PMID:15157725 Sources: GOC:cls, GOC:dgh, GOC:dph, GOC:jid, GO_REF:0000021 Definition: The migration of postmitotic a Purkinje cell along radial glial cells from the ventricular zone to the Purkinje cell layer. Relationships: is a type of hindbrain radial glia guided cell migration [GO:0021932]